N-acetylglucosaminyl-proteoglycan 4-beta-glucuronosyltransferase activity [GO:0050509] (molecular function) Sources: EC:2.4.1.225, MetaCyc:2.4.1.225-RXN, RHEA:20908 Also known as: N-acetylglucosaminyl-proteoglycan 4-b-glucuronosyltransferase activity, N-acetylglucosaminylproteoglycan beta-1,4-glucuronyltransferase activity, UDP-alpha-D-glucuronate:N-acetyl-alpha-D-glucosaminyl-(1->4)-beta-D-glucuronosyl-proteoglycan 4-beta-glucuronosyltransferase activity, heparan glucuronyltransferase II activity Relationships: is a type of glucuronosyltransferase activity [GO:0015020] Definition: Catalysis of the reaction: 3-O-{alpha-D-GlcNAc-[(1->4)-beta-D-GlcA-(1->4)-alpha-D-GlcNAc](n)-(1->4)-beta-D-GlcA-(1->3)-beta-D-Gal-(1->3)-beta-D-Gal-(1->4)-beta-D-Xyl}-L-seryl-[protein] + UDP-alpha-D-glucuronate = 3-O-{[(1->4)-beta-D-GlcA-(1->4)-alpha-D-GlcNAc](n+1)-(1->4)-beta-D-GlcA-(1->3)-beta-D-Gal-(1->3)-beta-D-Gal-(1->4)-beta-D-Xyl}-L-seryl-[protein] + H+ + UDP.